{
  "gene_symbol": "MEST",
  "term_id": "UNKNOWN:0002",
  "term_label": "Unknown biological process",
  "gene_name": "Mesoderm-specific transcript homolog protein",
  "gene": "UniProtKB:Q5EB52"
}